{
  "gene_name": "Polypeptide N-acetylgalactosaminyltransferase 16",
  "term_label": "Golgi apparatus",
  "gene": "UniProtKB:Q8N428",
  "term_id": "GO:0005794",
  "gene_symbol": "GALNT16"
}